{
  "gene_name": "Protein phosphatase 1H",
  "term_id": "GO:0004741",
  "term_label": "[pyruvate dehydrogenase (acetyl-transferring)]-phosphatase activity",
  "gene": "UniProtKB:Q9ULR3",
  "gene_symbol": "PPM1H"
}